{
  "gene_name": "(Lyso)-N-acylphosphatidylethanolamine lipase",
  "term_label": "lysophosphatidic acid acyltransferase activity",
  "gene_symbol": "ABHD4",
  "gene": "UniProtKB:Q8TB40",
  "term_id": "GO:0042171"
}